isotype switching to IgA isotypes [GO:0048290] (biological process) Regulation: regulated by regulation of isotype switching to IgA isotypes [GO:0048296]; negatively regulated by negative regulation of isotype switching to IgA isotypes [GO:0048297]; positively regulated by positive regulation of isotype switching to IgA isotypes [GO:0048298] References: PMID:12370374, PMID:2113175, PMID:9186655 Sources: ISBN:0781735149 Definition: The switching of activated B cells from IgM biosynthesis to biosynthesis of an IgA isotype, accomplished through a recombination process involving an intrachromosomal deletion between switch regions that reside 5' of the IgM and one of the IgA constant region gene segments in the immunoglobulin heavy chain locus. Relationships: is a type of isotype switching [GO:0045190] Also known as: class switching to IgA isotypes, isotype switch recombination to IgA isotypes